{
  "term_id": "GO:0003713",
  "gene_symbol": "CITED1",
  "gene": "UniProtKB:Q99966",
  "gene_name": "Cbp_p300-interacting transactivator 1",
  "term_label": "transcription coactivator activity"
}